CMP-N-acetylneuraminate metabolic process [GO:0046381] (biological process) Definition: The chemical reactions and pathways involving CMP-N-acetylneuraminate, a substance composed of 5-(acetylamino)-3,5-dideoxy-D-glycero-D-galacto-non-3-ulosonic acid in glycosidic linkage with cytidine monophosphate. Sources: GOC:ai Relationships: is a type of nucleotide-sugar metabolic process [GO:0009225] Subtypes: CMP-N-acetylneuraminate biosynthetic process [GO:0006055] Also known as: CMP-N-acetylneuraminate metabolism